prolactin signaling pathway [GO:0038161] (biological process) Definition: The series of molecular signals initiated by the binding of the peptide hormone prolactin to its receptor on the surface of a target cell, and ending with the regulation of a downstream cellular process, e.g. transcription. Also known as: PRL signaling pathway, prolactin-mediated signaling pathway References: PMID:21664429 Sources: GOC:nhn, GOC:signaling Regulation: regulated by regulation of prolactin signaling pathway [GO:1902211]; negatively regulated by negative regulation of prolactin signaling pathway [GO:1902212]; positively regulated by GO:1902213 Relationships: is_a hormone-mediated signaling pathway [GO:0009755]; is_a GO:0019221